{
  "term_label": "cytoplasm",
  "gene_name": "Proto-oncogene FRAT1",
  "gene": "UniProtKB:Q92837",
  "gene_symbol": "FRAT1",
  "term_id": "GO:0005737"
}